{
  "gene": "UniProtKB:P0DMV9",
  "gene_symbol": "HSPA1B",
  "gene_name": "Heat shock 70 kDa protein 1B",
  "term_id": "GO:0016887",
  "term_label": "ATP hydrolysis activity"
}